{
  "term_label": "Unknown biological process",
  "gene_name": "Protein MFI",
  "gene_symbol": "MFI",
  "term_id": "UNKNOWN:0002",
  "gene": "UniProtKB:Q8NCR3"
}